toll-like receptor TLR6:TLR2 signaling pathway [GO:0038124] (biological process) Also known as: TLR2:TLR6 signaling pathway, toll-like receptor TLR6:TLR2 signalling pathway Definition: The series of molecular signals initiated by a ligand binding of a heterodimeric TLR6:TLR2 complex, followed by transmission of the signal by the activated receptor, and ending with the regulation of a downstream cellular process, e.g. transcription. References: PMID:17318230 Sources: GOC:nhn, GOC:signaling Relationships: is a type of GO:0002224